{
  "term_label": "G1/S transition of mitotic cell cycle",
  "gene_symbol": "CCNB1",
  "gene_name": "G2_mitotic-specific cyclin-B1",
  "gene": "UniProtKB:P14635",
  "term_id": "GO:0000082"
}